{
  "gene_name": "Keratin-associated protein 2-1",
  "gene": "UniProtKB:Q9BYU5",
  "term_id": "UNKNOWN:0003",
  "gene_symbol": "KRTAP2-1",
  "term_label": "Unknown cellular component"
}